{
  "gene_name": "Oxysterol-binding protein-related protein 9",
  "term_id": "GO:0005829",
  "term_label": "cytosol",
  "gene_symbol": "OSBPL9",
  "gene": "UniProtKB:Q96SU4"
}